trehalose:proton symporter activity [GO:0044693] (molecular function) Relationships: is_a GO:0005351; is a type of trehalose transmembrane transporter activity [GO:0015574] Definition: Enables the transfer of a solute or solutes from one side of a membrane to the other according to the reaction: trehalose(out) + H+(out) = trehalose(in) + H+(in). Also known as: trehalose:hydrogen symporter activity References: PMID:11136464